{
  "gene_symbol": "LYPLA2",
  "gene": "UniProtKB:O95372",
  "term_id": "GO:1905344",
  "gene_name": "Acyl-protein thioesterase 2",
  "term_label": "prostaglandin catabolic process"
}